{
  "term_id": "GO:0000828",
  "term_label": "inositol hexakisphosphate kinase activity",
  "gene_name": "Inositol hexakisphosphate kinase 2",
  "gene": "UniProtKB:Q9UHH9",
  "gene_symbol": "IP6K2"
}